{
  "term_label": "mitochondrion",
  "term_id": "GO:0005739",
  "gene_name": "Monofunctional C1-tetrahydrofolate synthase, mitochondrial",
  "gene": "UniProtKB:Q6UB35",
  "gene_symbol": "MTHFD1L"
}